CKM complex [GO:1990508] (cellular component) Definition: Cyclin-dependent kinase complex which reversibly associates with the Mediator complex. In Saccharomyces cerevisiae it consists of SSN2, SSN3, SSN8 and SRB8. References: PMID:12200444 Sources: GOC:bhm Also known as: CDK8 kinase module, SRB8-SRB11 complex, SRB8/9/10/11 complex Note: An example of this is SSN2 in Saccharomyces cerevisiae (P38931) in PMID:12200444 (inferred from physical interaction). Relationships: is a type of nuclear cyclin-dependent protein kinase holoenzyme complex [GO:0019908]